{
  "gene_symbol": "LDB3",
  "term_label": "actin cytoskeleton organization",
  "term_id": "GO:0030036",
  "gene": "UniProtKB:O75112",
  "gene_name": "LIM domain-binding protein 3"
}